{
  "term_label": "GABA-A receptor complex",
  "gene": "UniProtKB:P47869",
  "gene_symbol": "GABRA2",
  "gene_name": "Gamma-aminobutyric acid receptor subunit alpha-2",
  "term_id": "GO:1902711"
}